{
  "gene": "UniProtKB:Q16445",
  "term_label": "synaptic transmission, GABAergic",
  "term_id": "GO:0051932",
  "gene_name": "Gamma-aminobutyric acid receptor subunit alpha-6",
  "gene_symbol": "GABRA6"
}